GUA codon-amino acid adaptor activity [GO:0033451] (molecular function) Sources: GOC:mah Relationships: is a type of triplet codon-amino acid adaptor activity [GO:0030533] Definition: A triplet codon-amino acid adaptor activity that recognizes a GUA codon. Note: Note that in the standard genetic code, GTA codes for valine. Also known as: GTA codon-amino acid adaptor activity, valine tRNA